{
  "gene": "UniProtKB:Q86Y39",
  "gene_symbol": "NDUFA11",
  "term_id": "UNKNOWN:0001",
  "gene_name": "NADH dehydrogenase [ubiquinone] 1 alpha subcomplex subunit 11",
  "term_label": "Unknown molecular function"
}